2'-5'-oligoadenylate synthetase activity [GO:0001730] (molecular function) Relationships: is a type of adenylyltransferase activity [GO:0070566] Definition: Catalysis of the reaction: ATP = pppA(2'p5'A)n oligomers. This reaction requires the binding of double-stranded RNA. Sources: ISBN:0198506732 Also known as: (2-5')oligo(A) synthetase activity, 2'-5' oligoadenylate synthetase activity, 2-5A synthetase activity, oligo-2',5'-adenylate synthetase activity